chromoplast stroma [GO:0009575] (cellular component) Relationships: is a type of plastid stroma [GO:0009532]; is part of GO:0009509 Sources: GOC:jl Definition: The space enclosed by the double membrane of a chromoplast but excluding the photosynthetic material.